left ventricular trabecular myocardium morphogenesis [GO:0003225] (biological process) Definition: The process in which the anatomical structures of cardiac left ventricular trabecular myocardium are generated and organized. Relationships: is a type of left ventricular cardiac muscle tissue morphogenesis [GO:0003220]; is a type of ventricular trabecula myocardium morphogenesis [GO:0003222] Sources: GOC:mtg_heart